{
  "term_id": "GO:0004984",
  "term_label": "olfactory receptor activity",
  "gene": "UniProtKB:Q9NZP2",
  "gene_symbol": "OR6C2",
  "gene_name": "Olfactory receptor 6C2"
}